{
  "gene": "UniProtKB:Q96DE9",
  "gene_name": "Protein EOLA2",
  "gene_symbol": "EOLA2",
  "term_label": "Unknown biological process",
  "term_id": "UNKNOWN:0002"
}